release of sequestered calcium ion into postsynaptic cytosol [GO:0099586] (biological process) Sources: GOC:dos Definition: The process in which calcium ions sequestered in the endoplasmic reticulum, Golgi apparatus or mitochondria are released into the postsynaptic cytosol. Relationships: is a type of release of sequestered calcium ion into cytosol [GO:0051209]; is a type of establishment of localization in cell [GO:0051649]; occurs in postsynapse [GO:0098794]